{
  "term_label": "Unknown biological process",
  "gene_name": "COP9 signalosome complex subunit 4",
  "term_id": "UNKNOWN:0002",
  "gene_symbol": "COPS4",
  "gene": "UniProtKB:Q9BT78"
}